phytosteroid biosynthetic process [GO:0016129] (biological process) Definition: The chemical reactions and pathways resulting in the formation of phytosteroids, steroids that differ from animal steroids in having substitutions at C24 and/or a double bond at C22. Phytosteroids are so named because they occur in higher plants; some, notably ergosterol, are also found in fungi. Sources: GOC:go_curators, GOC:mah, ISBN:0471331309 Also known as: phytosteroid anabolism, phytosteroid biosynthesis, phytosteroid formation, phytosteroid synthesis Relationships: is a type of GO:0006694 Subtypes: ergosterol biosynthetic process [GO:0006696], brassinosteroid biosynthetic process [GO:0016132]